{
  "gene": "UniProtKB:P16410",
  "gene_symbol": "CTLA4",
  "gene_name": "Cytotoxic T-lymphocyte protein 4",
  "term_id": "GO:0045590",
  "term_label": "negative regulation of regulatory T cell differentiation"
}